{
  "gene_name": "Bifunctional heparan sulfate N-deacetylase_N-sulfotransferase 3",
  "term_label": "heparan sulfate N-sulfotransferase activity",
  "term_id": "GO:0015016",
  "gene": "UniProtKB:O95803",
  "gene_symbol": "NDST3"
}